p-cresol biosynthetic process [GO:1901786] (biological process) Definition: The chemical reactions and pathways resulting in the formation of p-cresol. References: PMID:10623531 Sources: GOC:TermGenie, GOC:yaf Also known as: p-cresol anabolism, p-cresol biosynthesis, p-cresol formation, p-cresol synthesis Relationships: is a type of benzene-containing compound metabolic process [GO:0042537]; is a type of GO:0046189